{
  "term_id": "GO:0016020",
  "gene_name": "ABC-type oligopeptide transporter ABCB9",
  "term_label": "membrane",
  "gene_symbol": "ABCB9",
  "gene": "UniProtKB:Q9NP78"
}